{
  "gene_symbol": "MACROH2A2",
  "term_id": "GO:1901837",
  "gene_name": "Core histone macro-H2A.2",
  "gene": "UniProtKB:Q9P0M6",
  "term_label": "negative regulation of transcription of nucleolar large rRNA by RNA polymerase I"
}